{
  "term_id": "GO:0030154",
  "term_label": "cell differentiation",
  "gene_symbol": "NANOGP8",
  "gene": "UniProtKB:Q6NSW7",
  "gene_name": "Homeobox protein NANOGP8"
}